{
  "term_label": "Unknown molecular function",
  "gene_name": "Uncharacterized protein",
  "term_id": "UNKNOWN:0001",
  "gene": "UniProtKB:A0A3B3IRQ3",
  "gene_symbol": "LOC112267897"
}